{
  "gene": "UniProtKB:Q6NXP6",
  "gene_symbol": "NOXRED1",
  "gene_name": "NADP-dependent oxidoreductase domain-containing protein 1",
  "term_label": "L-proline biosynthetic process",
  "term_id": "GO:0055129"
}